{
  "term_id": "GO:0006357",
  "gene_symbol": "ZNF709",
  "term_label": "regulation of transcription by RNA polymerase II",
  "gene": "UniProtKB:Q8N972",
  "gene_name": "Zinc finger protein 709"
}